{
  "gene_name": "Nuclear distribution protein nudE homolog 1",
  "term_id": "GO:0007100",
  "term_label": "mitotic centrosome separation",
  "gene_symbol": "NDE1",
  "gene": "UniProtKB:Q9NXR1"
}